{
  "term_id": "GO:0007186",
  "term_label": "G protein-coupled receptor signaling pathway",
  "gene": "UniProtKB:A6NL26",
  "gene_name": "Olfactory receptor 5B21",
  "gene_symbol": "OR5B21"
}